embryonic plasmatocyte differentiation [GO:0035164] (biological process) Relationships: is a type of embryonic hemocyte differentiation [GO:0035163]; is a type of GO:0042387 Also known as: embryonic plasmatocyte cell differentiation References: PMID:11921077, PMID:8174791 Sources: GOC:bf Definition: The process in which an embryonic mesoderm-derived hemocyte precursor cell acquires the specialized features of the phagocytic blood-cell type, the plasmatocyte.